{
  "gene_symbol": "JAKMIP1",
  "gene": "UniProtKB:Q96N16",
  "gene_name": "Janus kinase and microtubule-interacting protein 1",
  "term_label": "GABA receptor binding",
  "term_id": "GO:0050811"
}